{
  "gene_name": "Tyrosine-protein kinase receptor UFO",
  "gene": "UniProtKB:P30530",
  "gene_symbol": "AXL",
  "term_label": "platelet activation",
  "term_id": "GO:0030168"
}